{
  "gene_name": "Complement component C8 gamma chain",
  "gene": "UniProtKB:P07360",
  "term_id": "UNKNOWN:0001",
  "gene_symbol": "C8G",
  "term_label": "Unknown molecular function"
}